{
  "gene": "UniProtKB:P13667",
  "term_label": "protein disulfide isomerase activity",
  "gene_symbol": "PDIA4",
  "gene_name": "Protein disulfide-isomerase A4",
  "term_id": "GO:0003756"
}